{
  "gene_symbol": "VAMP4",
  "gene": "UniProtKB:O75379",
  "term_id": "GO:0031201",
  "term_label": "SNARE complex",
  "gene_name": "Vesicle-associated membrane protein 4"
}